{
  "term_id": "GO:0005886",
  "term_label": "plasma membrane",
  "gene": "UniProtKB:Q96A23",
  "gene_symbol": "CPNE4",
  "gene_name": "Copine-4"
}